{
  "gene_symbol": "SLC4A2",
  "term_id": "GO:0051453",
  "gene": "UniProtKB:P04920",
  "gene_name": "Anion exchange protein 2",
  "term_label": "regulation of intracellular pH"
}